{
  "gene": "UniProtKB:P22532",
  "gene_symbol": "SPRR2D",
  "term_id": "UNKNOWN:0003",
  "term_label": "Unknown cellular component",
  "gene_name": "Small proline-rich protein 2D"
}